{
  "gene_symbol": "DCP2",
  "gene_name": "m7GpppN-mRNA hydrolase",
  "term_label": "cytoplasm",
  "term_id": "GO:0005737",
  "gene": "UniProtKB:Q8IU60"
}